{
  "gene_symbol": "ANKMY2",
  "term_label": "Unknown molecular function",
  "gene": "UniProtKB:Q8IV38",
  "gene_name": "Ankyrin repeat and MYND domain-containing protein 2",
  "term_id": "UNKNOWN:0001"
}